{
  "term_id": "GO:0018279",
  "gene_symbol": "UGGT2",
  "gene": "UniProtKB:Q9NYU1",
  "gene_name": "UDP-glucose:glycoprotein glucosyltransferase 2",
  "term_label": "protein N-linked glycosylation via asparagine"
}